RNA polymerase III type 1 promoter sequence-specific DNA binding [GO:0001002] (molecular function) References: PMID:12381659 Sources: GOC:txnOH Relationships: is a type of RNA polymerase III cis-regulatory region sequence-specific DNA binding [GO:0000992]; is a type of 5S rDNA binding [GO:0080084] Also known as: RNA polymerase III type 1 promoter DNA binding Definition: Binding to a sequence of DNA that is a part of a type 1 promoter that controls transcription by RNA polymerase III. Type 1 promoters are found in 5S rRNA genes, downstream of the transcription start site within the sequence of the mature RNA, and require TFIIIA for recognition.